{
  "gene_name": "Caspase-5",
  "gene_symbol": "CASP5",
  "term_label": "cytosol",
  "term_id": "GO:0005829",
  "gene": "UniProtKB:P51878"
}